{
  "term_label": "cytoplasm",
  "gene_symbol": "TESPA1",
  "term_id": "GO:0005737",
  "gene": "UniProtKB:A2RU30",
  "gene_name": "Protein TESPA1"
}